{
  "gene": "UniProtKB:Q6ZU15",
  "term_id": "GO:0032153",
  "gene_name": "Septin-14",
  "gene_symbol": "SEPTIN14",
  "term_label": "cell division site"
}